negative regulation of cytokine activity [GO:0060302] (biological process) Relationships: is a type of negative regulation of signal transduction [GO:0009968]; is a type of GO:0060300; is a type of negative regulation of receptor binding [GO:1900121]; negatively regulates cytokine activity [GO:0005125] Sources: GOC:BHF, GOC:dph, GOC:tb Definition: Any process that decreases the rate, frequency or extent of the activity of a molecule that controls the survival, growth, differentiation and effector function of tissues and cells. Subtypes: negative regulation of chemokine activity [GO:1900137]